peptidoglycan-based cell wall biogenesis [GO:0009273] (BP) Sources: GOC:go_curators Relationships: is a type of cell wall biogenesis [GO:0042546] Definition: The chemical reactions and pathways resulting in the formation of the peptidoglycan-based cell wall. An example of this process is found in Escherichia coli. Also known as: cell envelope biosynthesis, cell envelope biosynthetic process, cell wall anabolism, cell wall assembly, cell wall biosynthetic process, cell wall formation, cell wall synthesis Subtypes: Gram-negative-bacterium-type cell wall biogenesis [GO:0043164], Actinobacterium-type cell wall biogenesis [GO:0071766]